photoperiodism, flowering [GO:0048573] (biological process) Definition: A change from the vegetative to the reproductive phase as a result of detection of, or exposure to, a period of light or dark of a given length. The length of the period of light or dark required to initiate the change is set relative to a particular duration known as the 'critical day length'. The critical day length varies between species. Sources: GOC:jid, GOC:pj, ISBN:0582015952, ISBN:0697037754, ISBN:0709408862 Also known as: photoperiodic control of flowering time, photoperiodic control of inflorescence development, response to day length, flowering, response to night length, flowering, response to photoperiod, flowering Relationships: is a type of photoperiodism [GO:0009648]; is part of vegetative to reproductive phase transition of meristem [GO:0010228] Subtypes: long-day photoperiodism, flowering [GO:0048574], short-day photoperiodism, flowering [GO:0048575] Regulation: RO_0002211 by regulation of photoperiodism, flowering [GO:2000028]